{
  "term_id": "GO:0009306",
  "gene": "UniProtKB:Q9UBF2",
  "gene_symbol": "COPG2",
  "gene_name": "Coatomer subunit gamma-2",
  "term_label": "protein secretion"
}